regulation of lens fiber cell differentiation [GO:1902746] (biological process) Also known as: regulation of lens fibre cell differentiation References: PMID:17592637 Sources: GOC:TermGenie, GOC:mr, GO_REF:0000058 Definition: Any process that modulates the frequency, rate or extent of lens fiber cell differentiation. Relationships: is a type of regulation of epithelial cell differentiation [GO:0030856]; regulates GO:0070306 Subtypes: negative regulation of lens fiber cell differentiation [GO:1902747], GO:1902748